{
  "term_label": "long-chain fatty acid import into peroxisome",
  "gene": "UniProtKB:Q9UBJ2",
  "gene_symbol": "ABCD2",
  "term_id": "GO:0015910",
  "gene_name": "ATP-binding cassette sub-family D member 2"
}